{
  "term_id": "GO:0006457",
  "gene": "UniProtKB:Q8N807",
  "gene_symbol": "PDILT",
  "term_label": "protein folding",
  "gene_name": "Protein disulfide-isomerase-like protein of the testis"
}